limb epidermis stratification [GO:0060888] (biological process) Sources: GOC:dph, GOC:sdb_2009, GOC:tb Relationships: is a type of GO:0003002; is a type of limb epidermis development [GO:0060887] Definition: The pattern specification process that results in the subdivision of the epidermis of the limb in space to define a volume in which specific patterns of basal cell, spinous cell and granular cells will differentiate giving rise to the layers of the limb epidermis.